{
  "gene": "UniProtKB:Q9Y2E5",
  "term_id": "GO:0005764",
  "gene_symbol": "MAN2B2",
  "gene_name": "Epididymis-specific alpha-mannosidase",
  "term_label": "lysosome"
}